{
  "term_id": "UNKNOWN:0001",
  "gene_symbol": "SURF2",
  "gene_name": "Surfeit locus protein 2",
  "gene": "UniProtKB:Q15527",
  "term_label": "Unknown molecular function"
}